histone H3K27ac reader activity [GO:0140119] (molecular function) Relationships: is a type of GO:0140006 Definition: A histone reader that recognizes a histone H3 acetylated at lysine 27. Also known as: histone H3K27ac modified histone binding Note: Comment: Note that the residue position corresponds to the canonical human H3 histone (UniProtKB:P84243); this residue is conserved across all eukaryotes. Residue 1 is the first residue following removal of the initiating Methionine (Met). Note that each histone is encoded by multiple genes, and sequences may vary across different genes within an organism. References: PMID:25417107